{
  "gene_name": "Transformation_transcription domain-associated protein",
  "gene": "UniProtKB:Q9Y4A5",
  "term_label": "DNA repair-dependent chromatin remodeling",
  "gene_symbol": "TRRAP",
  "term_id": "GO:0140861"
}